thromboxane A2 signaling pathway [GO:0038193] (biological process) Relationships: is a type of G protein-coupled receptor signaling pathway [GO:0007186] Definition: A G protein-coupled receptor signaling pathway initiated by thromboxane A2 binding to its receptor on the surface of a target cell, and ending with the regulation of a downstream cellular process, e.g. transcription. References: PMID:15893915 Sources: GOC:nhn Also known as: TXA(2) receptor signaling, TXA2 signaling